Golgi apparatus [GO:0005794] (cellular component) Relationships: is a type of intracellular membrane-bounded organelle [GO:0043231]; is part of cytoplasm [GO:0005737]; is part of endomembrane system [GO:0012505] Note: Note that the Golgi apparatus can be located in various places in the cytoplasm. In plants and lower animal cells, the Golgi apparatus exists as many copies of discrete stacks dispersed throughout the cytoplasm, while the Golgi apparatus of interphase mammalian cells is a juxtanuclear, often pericentriolar reticulum, where the discrete Golgi stacks are stitched together to form a compact and interconnected ribbon, sometimes called the Golgi ribbon. Also known as: Golgi, Golgi complex, Golgi ribbon Subtypes: GO:0150051 References: PMID:9695800 Sources: ISBN:0198506732 Definition: A membrane-bound cytoplasmic organelle of the endomembrane system that further processes the core oligosaccharides (e.g. N-glycans) added to proteins in the endoplasmic reticulum and packages them into membrane-bound vesicles. The Golgi apparatus operates at the intersection of the secretory, lysosomal, and endocytic pathways.